{
  "gene": "UniProtKB:P12838",
  "term_id": "GO:0050830",
  "gene_name": "Defensin alpha 4",
  "term_label": "defense response to Gram-positive bacterium",
  "gene_symbol": "DEFA4"
}